startle response [GO:0001964] (biological process) Relationships: is a type of response to external stimulus [GO:0009605]; is a type of neuromuscular process [GO:0050905] Definition: An action or movement due to the application of a sudden unexpected stimulus. Sources: GOC:dph